{
  "gene_name": "UL16-binding protein 3",
  "gene_symbol": "ULBP3",
  "term_id": "GO:0002486",
  "gene": "UniProtKB:Q9BZM4",
  "term_label": "antigen processing and presentation of endogenous peptide antigen via MHC class I via ER pathway, TAP-independent"
}